inositol-1,3,4,6-tetrakisphosphate 5-kinase activity [GO:0047326] (MF) Definition: Catalysis of the reaction: 1D-myo-inositol 1,3,4,6-tetrakisphosphate + ATP = 1D-myo-inositol 1,3,4,5,6-pentakisphosphate + ADP + H+. Also known as: 1D-myo-inositol-tetrakisphosphate 5-kinase activity, inositol tetrakisphosphate 5-kinase activity, inositol-tetrakisphosphate 5-kinase activity, inositol 1,3,4,6-tetrakisphosphate 5-kinase activity, ATP:1D-myo-inositol-1,3,4,6-tetrakisphosphate 5-phosphotransferase activity Sources: RHEA:12717 Relationships: is a type of GO:0051765